{
  "gene_symbol": "CHST2",
  "gene": "UniProtKB:Q9Y4C5",
  "term_label": "sulfur compound metabolic process",
  "gene_name": "Carbohydrate sulfotransferase 2",
  "term_id": "GO:0006790"
}